{
  "gene": "UniProtKB:Q8NEU8",
  "gene_name": "DCC-interacting protein 13-beta",
  "term_id": "UNKNOWN:0001",
  "term_label": "Unknown molecular function",
  "gene_symbol": "APPL2"
}